peptide pheromone export [GO:0000770] (biological process) Definition: The directed movement of a peptide pheromone out of a cell by a secretion or export pathway used solely for the export of peptide pheromones. Sources: GOC:elh Also known as: a-factor export Relationships: is a type of GO:0042886 Subtypes: peptide pheromone secretion [GO:0090538], peptide pheromone export by transmembrane transport [GO:0090539]